glycine biosynthetic process from serine [GO:0019264] (biological process) Sources: GOC:go_curators Also known as: glycine anabolism from serine, glycine formation from serine, glycine synthesis from serine Definition: The chemical reactions and pathways resulting in the formation of glycine from other compounds, including serine. Relationships: is a type of glycine biosynthetic process [GO:0006545]; is a type of L-serine metabolic process [GO:0006563]